negative regulation of prolactin secretion [GO:1902721] (biological process) Definition: Any process that stops, prevents or reduces the frequency, rate or extent of prolactin secretion. References: PMID:16159377 Sources: GOC:TermGenie, GO_REF:0000058 Also known as: down regulation of prolactin secretion, down-regulation of prolactin secretion, downregulation of prolactin secretion, inhibition of prolactin secretion Relationships: is a type of negative regulation of protein secretion [GO:0050709]; is a type of negative regulation of peptide hormone secretion [GO:0090278]; negatively regulates GO:0070459